{
  "gene_name": "Fc receptor-like protein 5",
  "gene": "UniProtKB:Q96RD9",
  "term_id": "GO:0007166",
  "term_label": "cell surface receptor signaling pathway",
  "gene_symbol": "FCRL5"
}